metanephric glomerulus morphogenesis [GO:0072275] (biological process) Definition: The process in which the anatomical structures of the metanephric glomerulus are generated and organized. The metanephric glomerulus is a capillary tuft surrounded by Bowman's capsule in nephrons of the vertebrate kidney, or metanephros. Relationships: is a type of glomerulus morphogenesis [GO:0072102]; is part of metanephric glomerulus development [GO:0072224] Sources: GOC:mtg_kidney_jan10